smoothened binding [GO:0005119] (molecular function) Definition: Binding to a smoothened (smo) protein, which interacts with patched to transmit hedgehog signals. Relationships: is a type of GO:0001664 References: PMID:11731473 Sources: GOC:ceb Also known as: smo binding, smo ligand, smoothened ligand